{
  "term_label": "Unknown cellular component",
  "gene": "UniProtKB:O95236",
  "gene_symbol": "APOL3",
  "term_id": "UNKNOWN:0003",
  "gene_name": "Apolipoprotein L3"
}